{
  "gene_symbol": "PRKCD",
  "term_id": "GO:0004674",
  "gene_name": "Protein kinase C delta type",
  "term_label": "protein serine/threonine kinase activity",
  "gene": "UniProtKB:Q05655"
}